mitochondrial tRNA threonylcarbamoyladenosine modification [GO:0072670] (BP) Definition: The attachment of a carbonyl group and a threonine to the amino group of the adenine residue immediately 3' of the anticodon, in mitochondrial tRNAs that decode ANN codons (where N is any base). References: PMID:21183954 Sources: GOC:mcc Relationships: is a type of GO:0002949; is a type of mitochondrial tRNA modification [GO:0070900] Also known as: mitochondrial tRNA t6A modification